{
  "term_label": "Unknown molecular function",
  "gene": "UniProtKB:Q9UK00",
  "gene_name": "Uncharacterized protein C3orf18",
  "term_id": "UNKNOWN:0001",
  "gene_symbol": "C3orf18"
}